{
  "gene_name": "Potassium voltage-gated channel subfamily KQT member 1",
  "term_id": "GO:0001508",
  "gene": "UniProtKB:P51787",
  "term_label": "action potential",
  "gene_symbol": "KCNQ1"
}